response to diethyl maleate [GO:1902111] (biological process) Relationships: is_a GO:1901700 References: PMID:12100563 Sources: GOC:TermGenie Definition: Any process that results in a change in state or activity of a cell or an organism (in terms of movement, secretion, enzyme production, gene expression, etc.) as a result of a diethyl maleate stimulus. Subtypes: cellular response to diethyl maleate [GO:1902112]